{
  "term_label": "DNA helicase activity",
  "gene": "UniProtKB:Q13283",
  "gene_symbol": "G3BP1",
  "term_id": "GO:0003678",
  "gene_name": "Ras GTPase-activating protein-binding protein 1"
}